{
  "gene": "UniProtKB:A6NLU0",
  "gene_symbol": "RFPL4A",
  "term_id": "GO:0061630",
  "gene_name": "Ret finger protein-like 4A",
  "term_label": "ubiquitin protein ligase activity"
}